{
  "gene": "UniProtKB:Q0D2K0",
  "gene_symbol": "NIPAL4",
  "gene_name": "Magnesium transporter NIPA4",
  "term_id": "GO:0016020",
  "term_label": "membrane"
}